{
  "term_label": "Unknown biological process",
  "gene_name": "SAP30-binding protein",
  "term_id": "UNKNOWN:0002",
  "gene_symbol": "SAP30BP",
  "gene": "UniProtKB:Q9UHR5"
}